{
  "term_label": "Unknown biological process",
  "gene_name": "Paraneoplastic antigen-like protein 8C",
  "term_id": "UNKNOWN:0002",
  "gene": "UniProtKB:A0A1B0GUJ8",
  "gene_symbol": "PNMA8C"
}